intracellular monoatomic ion homeostasis [GO:0006873] (biological process) Relationships: is a type of GO:0050801; is a type of intracellular chemical homeostasis [GO:0055082] Also known as: cellular ion homeostasis, cellular monoatomic ion homeostasis Subtypes: intracellular monoatomic anion homeostasis [GO:0030002], GO:0030003 Definition: A homeostatic process involved in the maintenance of a steady state level of monoatomic ions within a cell. Monatomic ions (also called simple ions) are ions consisting of exactly one atom. Sources: GOC:mah